{
  "term_label": "cytoplasm",
  "gene_symbol": "ARAP2",
  "term_id": "GO:0005737",
  "gene_name": "Arf-GAP with Rho-GAP domain, ANK repeat and PH domain-containing protein 2",
  "gene": "UniProtKB:Q8WZ64"
}